{
  "gene": "UniProtKB:Q8NGN5",
  "gene_symbol": "OR10G8",
  "term_id": "GO:0005886",
  "gene_name": "Olfactory receptor 10G8",
  "term_label": "plasma membrane"
}